response to vitamin K [GO:0032571] (biological process) Subtypes: response to menaquinone [GO:0032572], GO:0032573, cellular response to vitamin K [GO:0071307] Definition: Any process that results in a change in state or activity of a cell or an organism (in terms of movement, secretion, enzyme production, gene expression, etc.) as a result of a vitamin K stimulus. Relationships: is a type of GO:0033273; is a type of response to ketone [GO:1901654] Sources: GOC:sl